{
  "gene": "UniProtKB:O43657",
  "gene_name": "Tetraspanin-6",
  "term_id": "GO:0005886",
  "gene_symbol": "TSPAN6",
  "term_label": "plasma membrane"
}